{
  "gene": "UniProtKB:Q9NZH0",
  "gene_symbol": "GPRC5B",
  "term_label": "protein kinase binding",
  "term_id": "GO:0019901",
  "gene_name": "G-protein coupled receptor family C group 5 member B"
}